{
  "term_label": "Unknown molecular function",
  "gene_symbol": "DNAAF11",
  "gene_name": "Dynein axonemal assembly factor 11",
  "gene": "UniProtKB:Q86X45",
  "term_id": "UNKNOWN:0001"
}